{
  "gene_symbol": "RUNX3",
  "gene_name": "Runt-related transcription factor 3",
  "term_id": "GO:0006357",
  "term_label": "regulation of transcription by RNA polymerase II",
  "gene": "UniProtKB:Q13761"
}